interleukin-25 receptor binding [GO:0045521] (molecular function) Sources: GOC:go_curators Definition: Binding to an interleukin-25 receptor. Relationships: is a type of GO:0005126 Also known as: IL-25, interleukin-25 receptor ligand